{
  "gene": "UniProtKB:Q9UPW0",
  "gene_name": "Forkhead box protein J3",
  "term_label": "nucleus",
  "term_id": "GO:0005634",
  "gene_symbol": "FOXJ3"
}